6-phospho-3-hexuloisomerase activity [GO:0043800] (molecular function) Also known as: HUMPI, hexulose-6-phosphate isomerase activity Relationships: is a type of intramolecular oxidoreductase activity, interconverting aldoses and ketoses [GO:0016861] References: PMID:11839305 Sources: RHEA:25900 Definition: Catalysis of the reaction: D-arabino-hex-3-ulose 6-phosphate = beta-D-fructose 6-phosphate.